{
  "gene_name": "Polypeptide N-acetylgalactosaminyltransferase 16",
  "term_id": "GO:0006493",
  "gene_symbol": "GALNT16",
  "term_label": "protein O-linked glycosylation",
  "gene": "UniProtKB:Q8N428"
}